{
  "gene_name": "Sorting nexin-16",
  "gene": "UniProtKB:P57768",
  "term_id": "GO:0045022",
  "gene_symbol": "SNX16",
  "term_label": "early endosome to late endosome transport"
}